{
  "gene": "UniProtKB:P10909",
  "gene_name": "Clusterin",
  "term_id": "GO:0042981",
  "term_label": "regulation of apoptotic process",
  "gene_symbol": "CLU"
}